{
  "term_label": "extracellular space",
  "gene_name": "Attractin",
  "gene": "UniProtKB:O75882",
  "gene_symbol": "ATRN",
  "term_id": "GO:0005615"
}